{
  "gene_symbol": "SESN2",
  "term_label": "positive regulation of macroautophagy",
  "gene": "UniProtKB:P58004",
  "gene_name": "Sestrin-2",
  "term_id": "GO:0016239"
}